{
  "gene_symbol": "UBP1",
  "term_id": "GO:0000978",
  "term_label": "RNA polymerase II cis-regulatory region sequence-specific DNA binding",
  "gene": "UniProtKB:Q9NZI7",
  "gene_name": "Upstream-binding protein 1"
}